{
  "gene_symbol": "MTRNR2L11",
  "term_label": "receptor antagonist activity",
  "term_id": "GO:0048019",
  "gene": "UniProtKB:S4R3Y5",
  "gene_name": "Humanin-like 11"
}